{
  "gene": "UniProtKB:Q08426",
  "gene_name": "Peroxisomal bifunctional enzyme",
  "term_id": "GO:0006635",
  "gene_symbol": "EHHADH",
  "term_label": "fatty acid beta-oxidation"
}